{
  "term_label": "cell-cell junction",
  "term_id": "GO:0005911",
  "gene_symbol": "MAGI1",
  "gene_name": "Membrane-associated guanylate kinase, WW and PDZ domain-containing protein 1",
  "gene": "UniProtKB:Q96QZ7"
}